{
  "term_label": "immune receptor activity",
  "gene_name": "Immunoglobulin subtype domain-containing protein",
  "gene": "UniProtKB:A0A5F9Z9Y6",
  "gene_symbol": "A0A5F9Z9Y6",
  "term_id": "GO:0140375"
}